{
  "term_id": "GO:0007032",
  "gene": "UniProtKB:Q9BTU6",
  "gene_symbol": "PI4K2A",
  "term_label": "endosome organization",
  "gene_name": "Phosphatidylinositol 4-kinase type 2-alpha"
}